{
  "gene": "UniProtKB:P05015",
  "term_id": "GO:0002323",
  "gene_name": "Interferon alpha-16",
  "term_label": "natural killer cell activation involved in immune response",
  "gene_symbol": "IFNA16"
}